proteoglycan catabolic process [GO:0030167] (biological process) Also known as: proteoglycan breakdown, proteoglycan catabolism, proteoglycan degradation Subtypes: GO:0030200, chondroitin sulfate proteoglycan catabolic process [GO:0030207], GO:0030209, heparin proteoglycan catabolic process [GO:0030211], GO:0042340 Definition: The chemical reactions and pathways resulting in the breakdown of proteoglycans, any glycoprotein in which the carbohydrate units are glycosaminoglycans. Relationships: is a type of proteoglycan metabolic process [GO:0006029]; is_a GO:0006516 References: PMID:35536982